{
  "term_id": "GO:0042073",
  "term_label": "intraciliary transport",
  "gene": "UniProtKB:Q9UPZ9",
  "gene_name": "Serine_threonine-protein kinase ICK",
  "gene_symbol": "CILK1"
}